{
  "gene": "UniProtKB:Q56P03",
  "gene_name": "E2F-associated phosphoprotein",
  "gene_symbol": "EAPP",
  "term_label": "Unknown molecular function",
  "term_id": "UNKNOWN:0001"
}